{
  "gene_symbol": "GSTO2",
  "term_id": "GO:0004364",
  "gene": "UniProtKB:Q9H4Y5",
  "gene_name": "Glutathione S-transferase omega-2",
  "term_label": "glutathione transferase activity"
}